proteasome regulatory particle, lid subcomplex [GO:0008541] (cellular component) Subtypes: nuclear proteasome regulatory particle, lid subcomplex [GO:0031613], cytosolic proteasome regulatory particle, lid subcomplex [GO:0031615] Relationships: is a type of GO:0032991; is part of GO:0005838 Definition: The subcomplex of the proteasome regulatory particle that forms the peripheral lid, which is added on top of the base subcomplex. Sources: GOC:rb